high voltage-gated calcium channel activity [GO:0008331] (molecular function) Definition: Enables the transmembrane transfer of a calcium ion by a high voltage-gated channel. A high voltage-gated channel is a channel whose open state is dependent on high voltage across the membrane in which it is embedded. References: PMID:16382099 Sources: GOC:mtg_transport, ISBN:0815340729 Also known as: high voltage gated calcium channel activity, high voltage-dependent calcium channel activity, L-type calcium channel, N-type calcium channel, P-type calcium channel, Q-type calcium channel Relationships: is a type of GO:0005245 Regulation: negatively regulated by negative regulation of high voltage-gated calcium channel activity [GO:1901842]; RO_0002213 by positive regulation of high voltage-gated calcium channel activity [GO:1901843]